response to cortisol [GO:0051414] (biological process) Relationships: is a type of response to glucocorticoid [GO:0051384]; is a type of GO:0097305; is a type of response to ketone [GO:1901654] Definition: Any process that results in a change in state or activity of a cell or an organism (in terms of movement, secretion, enzyme production, gene expression, etc.) as a result of a cortisol stimulus. Cortisol is the major natural glucocorticoid synthesized in the zona fasciculata of the adrenal cortex; it affects the metabolism of glucose, protein, and fats and has appreciable mineralocorticoid activity. It also regulates the immune system and affects many other functions. Subtypes: cellular response to cortisol stimulus [GO:0071387] Also known as: response to cortisol stimulus, response to hydrocortisone stimulus References: PMID:11276391 Sources: ISBN:0721662544